{
  "gene_symbol": "H2AL3",
  "gene": "UniProtKB:A0A3B3IU63",
  "gene_name": "Histone H2A-like 3",
  "term_id": "GO:0030527",
  "term_label": "structural constituent of chromatin"
}